generation of precursor metabolites and energy [GO:0006091] (biological process) Regulation: regulated by regulation of generation of precursor metabolites and energy [GO:0043467] Subtypes: glycolytic process [GO:0006096], NADPH regeneration [GO:0006740], pentose-phosphate shunt, non-oxidative branch [GO:0009052], photosynthesis, light harvesting [GO:0009765], energy derivation by oxidation of reduced inorganic compounds [GO:0015975], energy derivation by oxidation of organic compounds [GO:0015980], GO:0019431, photosynthesis, light reaction [GO:0019684], GO:0022900, GO:0061719, sulphoglycolysis [GO:0061722], GO:1902224 Definition: The chemical reactions and pathways resulting in the formation of precursor metabolites, substances from which energy is derived, and any process involved in the liberation of energy from these substances. Also known as: energy pathways, intermediary metabolism, metabolic energy generation Relationships: is_a metabolic process [GO:0008152] Sources: GOC:jl